{
  "gene_name": "G protein-coupled receptor associated sorting protein 3",
  "gene": "UniProtKB:Q6PI77",
  "term_id": "UNKNOWN:0002",
  "gene_symbol": "GPRASP3",
  "term_label": "Unknown biological process"
}